glucose-1-phosphate adenylyltransferase complex [GO:0010170] (cellular component) Definition: Complex that catalyzes the synthesis of ADP-glucose and pyrophosphate from glucose-1-phosphate and ATP. In plants, the complex is a heterotetramer composed of two types of subunits (small and large). In bacteria, the enzyme complex is composed of four identical subunits. References: PMID:12748181 Sources: GOC:tb Relationships: is a type of intracellular protein-containing complex [GO:0140535]; is_a adenylyltransferase complex [GO:1902503]